{
  "term_id": "GO:0007274",
  "gene_name": "Neuronal acetylcholine receptor subunit alpha-2",
  "gene_symbol": "CHRNA2",
  "gene": "UniProtKB:Q15822",
  "term_label": "neuromuscular synaptic transmission"
}